{
  "gene_symbol": "ABT1",
  "term_id": "GO:0034462",
  "gene_name": "Activator of basal transcription 1",
  "gene": "UniProtKB:Q9ULW3",
  "term_label": "small-subunit processome assembly"
}